gerfelin biosynthetic process [GO:1900578] (biological process) Sources: GOC:TermGenie, GOC:di Also known as: gerfelin anabolism, gerfelin biosynthesis, gerfelin formation, gerfelin synthesis Regulation: regulated by regulation of gerfelin biosynthetic process [GO:1900686]; negatively regulated by negative regulation of gerfelin biosynthetic process [GO:1900687]; positively regulated by GO:1900688 Relationships: is a type of catechol-containing compound biosynthetic process [GO:0009713]; is a type of benzene-containing compound metabolic process [GO:0042537]; is_a secondary metabolite biosynthetic process [GO:0044550]; is a type of carboxylic acid biosynthetic process [GO:0046394]; is a type of GO:1901503 Definition: The chemical reactions and pathways resulting in the formation of gerfelin.